{
  "term_label": "Unknown biological process",
  "term_id": "UNKNOWN:0002",
  "gene_symbol": "CHIC2",
  "gene_name": "Cysteine-rich hydrophobic domain-containing protein 2",
  "gene": "UniProtKB:Q9UKJ5"
}